{
  "term_id": "GO:0003724",
  "term_label": "RNA helicase activity",
  "gene_symbol": "DDX3Y",
  "gene_name": "ATP-dependent RNA helicase DDX3Y",
  "gene": "UniProtKB:O15523"
}